{
  "gene_name": "Glutaryl-CoA dehydrogenase, mitochondrial",
  "gene": "UniProtKB:Q92947",
  "term_label": "fatty-acyl-CoA binding",
  "term_id": "GO:0000062",
  "gene_symbol": "GCDH"
}